{
  "term_id": "GO:0033617",
  "term_label": "mitochondrial respiratory chain complex IV assembly",
  "gene_symbol": "COX19",
  "gene_name": "Cytochrome c oxidase assembly protein COX19",
  "gene": "UniProtKB:Q49B96"
}